{
  "gene_name": "DnaJ homolog subfamily A member 4",
  "gene_symbol": "DNAJA4",
  "term_id": "GO:0001671",
  "gene": "UniProtKB:Q8WW22",
  "term_label": "ATPase activator activity"
}